{
  "term_id": "GO:0007095",
  "gene_symbol": "CHEK1",
  "gene_name": "Serine_threonine-protein kinase Chk1",
  "gene": "UniProtKB:O14757",
  "term_label": "mitotic G2 DNA damage checkpoint signaling"
}